{
  "gene_symbol": "WASHC5",
  "gene_name": "WASH complex subunit 5",
  "term_label": "endosome organization",
  "term_id": "GO:0007032",
  "gene": "UniProtKB:Q12768"
}